{
  "term_id": "GO:0016020",
  "gene_name": "Protein FAM83B",
  "gene": "UniProtKB:Q5T0W9",
  "term_label": "membrane",
  "gene_symbol": "FAM83B"
}